{
  "gene_name": "Thiopurine S-methyltransferase",
  "gene": "UniProtKB:P51580",
  "term_label": "Unknown cellular component",
  "gene_symbol": "TPMT",
  "term_id": "UNKNOWN:0003"
}